{
  "gene_name": "Tumor protein p63-regulated gene 1-like protein",
  "gene_symbol": "TPRG1L",
  "term_label": "synaptic vesicle",
  "term_id": "GO:0008021",
  "gene": "UniProtKB:Q5T0D9"
}